{
  "term_id": "GO:0006955",
  "gene_name": "Immunoglobulin kappa variable 2-29",
  "term_label": "immune response",
  "gene_symbol": "IGKV2-29",
  "gene": "UniProtKB:A2NJV5"
}